{
  "term_id": "GO:1990165",
  "gene": "UniProtKB:Q7Z2E3",
  "gene_name": "Aprataxin",
  "gene_symbol": "APTX",
  "term_label": "single-strand break-containing DNA binding"
}